{
  "term_label": "mitochondrial matrix",
  "gene": "UniProtKB:Q5T440",
  "term_id": "GO:0005759",
  "gene_symbol": "IBA57",
  "gene_name": "Putative transferase CAF17, mitochondrial"
}